{
  "gene_symbol": "SLC24A2",
  "term_id": "GO:0070588",
  "gene_name": "Sodium_potassium_calcium exchanger 2",
  "term_label": "calcium ion transmembrane transport",
  "gene": "UniProtKB:Q9UI40"
}